plastid stroma [GO:0009532] (cellular component) Sources: ISBN:0943088399 Definition: The proteinaceous ground substance of plastids. Relationships: is a type of cellular anatomical structure [GO:0110165]; is part of plastid [GO:0009536] Subtypes: chloroplast stroma [GO:0009570], proplastid stroma [GO:0009571], GO:0009575, leucoplast stroma [GO:0009576], elaioplast stroma [GO:0009577], etioplast stroma [GO:0009578], cyanelle stroma [GO:0034060], gerontoplast stroma [GO:1905506]